clearance of foreign intracellular nucleic acids [GO:0099046] (BP) Sources: GO:dos Subtypes: clearance of foreign intracellular DNA [GO:0044355], clearance of foreign intracellular RNA [GO:0099047], GO:0099048 Definition: A defense process that protects an organism from DNA or RNA from an invading organism. Relationships: is a type of GO:0140546